{
  "term_id": "GO:0005634",
  "gene_symbol": "MT1B",
  "gene_name": "Metallothionein-1B",
  "gene": "UniProtKB:P07438",
  "term_label": "nucleus"
}